{
  "term_id": "UNKNOWN:0001",
  "gene": "UniProtKB:O75293",
  "gene_symbol": "GADD45B",
  "term_label": "Unknown molecular function",
  "gene_name": "Growth arrest and DNA damage-inducible protein GADD45 beta"
}